{
  "gene_name": "Lymphocyte expansion molecule",
  "gene_symbol": "LEXM",
  "gene": "UniProtKB:Q3ZCV2",
  "term_label": "Unknown biological process",
  "term_id": "UNKNOWN:0002"
}